{
  "gene_symbol": "ZNF215",
  "term_label": "DNA-binding transcription factor activity, RNA polymerase II-specific",
  "gene_name": "Zinc finger protein 215",
  "gene": "UniProtKB:Q9UL58",
  "term_id": "GO:0000981"
}